{
  "gene_symbol": "PKNOX1",
  "gene_name": "Homeobox protein PKNOX1",
  "term_id": "GO:0000978",
  "term_label": "RNA polymerase II cis-regulatory region sequence-specific DNA binding",
  "gene": "UniProtKB:P55347"
}